{
  "term_id": "UNKNOWN:0001",
  "term_label": "Unknown molecular function",
  "gene": "UniProtKB:Q13336",
  "gene_symbol": "SLC14A1",
  "gene_name": "Urea transporter 1"
}